{
  "gene": "UniProtKB:Q9NPQ8",
  "gene_name": "Synembryn-A",
  "term_id": "GO:0005085",
  "term_label": "guanyl-nucleotide exchange factor activity",
  "gene_symbol": "RIC8A"
}